{
  "gene_symbol": "IGHV5-51",
  "gene_name": "Immunoglobulin heavy variable 5-51",
  "gene": "UniProtKB:A0A0C4DH38",
  "term_label": "antigen binding",
  "term_id": "GO:0003823"
}